heparin proteoglycan metabolic process [GO:0030202] (biological process) Relationships: is a type of proteoglycan metabolic process [GO:0006029] Subtypes: heparin proteoglycan biosynthetic process [GO:0030210], heparin proteoglycan catabolic process [GO:0030211] Definition: The chemical reactions and pathways involving heparin proteoglycans, which consist of a core protein linked to a heparin glycosaminoglycan. The heparin chain is composed of the repeating disaccharide unit beta-(1,4)-N-acetyl-D-glucosamine-alpha-(1,4)-hexuronic acid, the former being either sulfated or deacetylated on its amino group as well as sulfated on one of its hydroxyl groups, and the latter being e a mixture of sulfated and nonsulfated D-glucuronic and L-iduronic acids. Heparin is similar to heparan sulfate but it contains more N-sulfate and O-sulfate groups. Heparin proteoglycans are stored selectively in the secretory granules of mammalian mast cells. References: PMID:22566225 Also known as: heparin metabolism, heparan sulfate metabolic process